{
  "gene_name": "DNA ligase 3",
  "term_id": "GO:0003910",
  "gene_symbol": "LIG3",
  "term_label": "DNA ligase (ATP) activity",
  "gene": "UniProtKB:P49916"
}